{
  "gene_name": "Protein SLFN14",
  "term_label": "Unknown cellular component",
  "gene_symbol": "SLFN14",
  "term_id": "UNKNOWN:0003",
  "gene": "UniProtKB:P0C7P3"
}